{
  "gene_name": "Transmembrane protein 272",
  "gene": "UniProtKB:A0A1B0GTI8",
  "term_label": "Unknown cellular component",
  "term_id": "UNKNOWN:0003",
  "gene_symbol": "TMEM272"
}